P-type silver transporter activity [GO:0015445] (molecular function) Sources: RHEA:14733 Definition: Enables the transfer of a solute or solutes from one side of a membrane to the other according to the reaction: ATP + H2O + Ag+(in) = ADP + phosphate + Ag+(out). Also known as: silver exporting ATPase activity, silver transmembrane transporter activity, phosphorylative mechanism, ATP phosphohydrolase (Ag+-exporting), Ag+-exporting ATPase activity, silver-exporting ATPase activity Relationships: is a type of silver ion transmembrane transporter activity [GO:0015080]; is a type of P-type ion transporter activity [GO:0015662]; is a type of GO:0019829